extrathymic T cell selection [GO:0045062] (biological process) Also known as: extrathymic T lymphocyte selection, extrathymic T-cell selection, extrathymic T-lymphocyte selection Relationships: is a type of T cell selection [GO:0045058]; is part of extrathymic T cell differentiation [GO:0033078] Subtypes: positive extrathymic T cell selection [GO:0045067], negative extrathymic T cell selection [GO:0045068] Definition: The process of T cell selection that occurs in extrathymic locations, often resulting T cells of distinct specificities from those selected in the thymus. References: PMID:7880383 Sources: ISBN:0781735149